natural killer cell differentiation involved in immune response [GO:0002325] (biological process) Note: Note that immunologists typically use the word 'development' to refer to cells of B or T cell lineages undergoing the process that GO describes as 'cell differentiation'. Also known as: NK cell differentiation during immune response, natural killer cell development involved in immune response, natural killer cell differentiation during immune response Definition: The process in which a naive natural killer cell acquires the specialized features of an effector natural killer T cell as part of an immune response. Regulation: regulated by regulation of natural killer cell differentiation involved in immune response [GO:0032826]; negatively regulated by negative regulation of natural killer cell differentiation involved in immune response [GO:0032827]; positively regulated by positive regulation of natural killer cell differentiation involved in immune response [GO:0032828] References: PMID:11698225 Sources: GOC:add Relationships: is a type of GO:0001779; is a type of lymphocyte activation involved in immune response [GO:0002285]